mitochondrial ncRNA surveillance [GO:0035945] (biological process) Definition: The set of processes involved in identifying and degrading defective or aberrant non-coding RNA transcripts (ncRNAs) within the mitochondrion. Also known as: mitochondrial aberrant ncRNA catabolic process, mitochondrial ncRNA quality control, mitochondrial non-coding RNA surveillance References: PMID:19864255 Sources: GOC:ans Relationships: is a type of GO:2000827